{
  "gene_symbol": "LY6G6E",
  "gene": "UniProtKB:A0A0B4J1T7",
  "term_id": "GO:0005886",
  "term_label": "plasma membrane",
  "gene_name": "Lymphocyte antigen 6 family member G6E"
}